{
  "term_id": "UNKNOWN:0003",
  "gene_symbol": "LINC01356",
  "term_label": "Unknown cellular component",
  "gene": "UniProtKB:Q8N9X3",
  "gene_name": "Putative uncharacterized protein encoded by LINC01356"
}